{
  "gene_name": "Uncharacterized aarF domain-containing protein kinase 5",
  "gene": "UniProtKB:Q3MIX3",
  "term_label": "Unknown biological process",
  "gene_symbol": "ADCK5",
  "term_id": "UNKNOWN:0002"
}